{
  "gene_name": "Prelamin-A_C",
  "gene": "UniProtKB:P02545",
  "gene_symbol": "LMNA",
  "term_label": "nuclear migration",
  "term_id": "GO:0007097"
}